{
  "gene": "UniProtKB:P07741",
  "gene_name": "Adenine phosphoribosyltransferase",
  "term_label": "cytoplasm",
  "gene_symbol": "APRT",
  "term_id": "GO:0005737"
}